regulation of type III interferon production [GO:0034344] (BP) Note: Note that IL-28A, IL-28B, and IL-29 are types of interferon-lambda. Definition: Any process that modulates the frequency, rate, or extent of type III interferon production. Interferon lambda is the only member of the type III interferon found so far. Subtypes: negative regulation of type III interferon production [GO:0034345], positive regulation of type III interferon production [GO:0034346] References: PMID:15546383, PMID:16734557 Sources: GOC:add, ISBN:0126896631 Relationships: is a type of GO:0001817; RO_0002211 type III interferon production [GO:0034343] Also known as: regulation of type III IFN production